lipid tube assembly involved in organelle fusion [GO:0060989] (biological process) Definition: The aggregation, arrangement and bonding together of a set of macromolecules to form a macromolecular complex that contains a tube of lipid surrounded by a protein coat involved in membrane shaping of vesicle membranes as organelles fuse. Relationships: is a type of lipid tube assembly [GO:0060988]; is part of organelle fusion [GO:0048284] Sources: GOC:ascb_2009, GOC:dph, GOC:tb Also known as: lipid tubulation involved in organelle fusion